regulation of G2/M transition of mitotic cell cycle [GO:0010389] (biological process) Relationships: is_a regulation of mitotic cell cycle phase transition [GO:1901990]; is a type of regulation of cell cycle G2/M phase transition [GO:1902749]; regulates GO:0000086 Also known as: regulation of mitotic entry Definition: Any signaling pathway that modulates the activity of a cell cycle cyclin-dependent protein kinase to modulate the switch from G2 phase to M phase of the mitotic cell cycle. References: PMID:17329565 Sources: GOC:mtg_cell_cycle Subtypes: positive regulation of G2/M transition of mitotic cell cycle [GO:0010971], negative regulation of G2/M transition of mitotic cell cycle [GO:0010972]